endothelin receptor signaling pathway [GO:0086100] (biological process) References: PMID:10977869 Sources: GOC:BHF, GOC:bf, GOC:mtg_cardiac_conduct_nov11 Definition: A G protein-coupled receptor signaling pathway initiated by endothelin binding to its receptor on the surface of a target cell, and ending with the regulation of a downstream cellular process, e.g. transcription. Subtypes: endothelin receptor signaling pathway involved in heart process [GO:0086101], GO:0160135 Relationships: is a type of G protein-coupled receptor signaling pathway [GO:0007186] Also known as: endothelin signaling pathway